{
  "gene_name": "Uncharacterized protein C2orf66",
  "gene": "UniProtKB:Q6UXQ4",
  "term_label": "Unknown biological process",
  "gene_symbol": "C2orf66",
  "term_id": "UNKNOWN:0002"
}